{
  "gene": "UniProtKB:Q5TFG8",
  "gene_name": "Zinc finger C2HC domain-containing protein 1B",
  "term_label": "Unknown cellular component",
  "gene_symbol": "ZC2HC1B",
  "term_id": "UNKNOWN:0003"
}